{
  "gene_name": "Serine protease hepsin",
  "gene": "UniProtKB:P05981",
  "term_label": "serine-type peptidase activity",
  "term_id": "GO:0008236",
  "gene_symbol": "HPN"
}